{
  "gene_name": "Glutamate receptor ionotropic, kainate 5",
  "gene": "UniProtKB:Q16478",
  "gene_symbol": "GRIK5",
  "term_id": "GO:0035249",
  "term_label": "synaptic transmission, glutamatergic"
}